{
  "term_id": "UNKNOWN:0002",
  "gene_symbol": "HEATR9",
  "gene": "UniProtKB:A2RTY3",
  "term_label": "Unknown biological process",
  "gene_name": "Protein HEATR9"
}